{
  "gene_name": "Prospero homeobox protein 1",
  "gene_symbol": "PROX1",
  "term_label": "DNA-binding transcription factor activity, RNA polymerase II-specific",
  "term_id": "GO:0000981",
  "gene": "UniProtKB:Q92786"
}